{
  "term_id": "GO:0005634",
  "term_label": "nucleus",
  "gene_name": "Ubinuclein-1",
  "gene": "UniProtKB:Q9NPG3",
  "gene_symbol": "UBN1"
}